stipitatonate decarboxylase activity [GO:0050296] (MF) Also known as: stipitatonate carboxy-lyase (decyclizing), stipitatonate carboxy-lyase (decyclizing, stipitatate-forming) Sources: EC:4.1.1.60, RHEA:13885 Relationships: is a type of carboxy-lyase activity [GO:0016831] Definition: Catalysis of the reaction: H2O + stipitatonate = CO2 + H+ + stipitatate.